{
  "term_id": "GO:0030497",
  "gene": "UniProtKB:Q9P035",
  "gene_symbol": "HACD3",
  "term_label": "fatty acid elongation",
  "gene_name": "Very-long-chain (3R)-3-hydroxyacyl-CoA dehydratase 3"
}